{
  "gene_name": "Fanconi anemia group I protein",
  "gene_symbol": "FANCI",
  "term_label": "Unknown cellular component",
  "term_id": "UNKNOWN:0003",
  "gene": "UniProtKB:Q9NVI1"
}